{
  "term_label": "cytoplasm",
  "gene_name": "Tubulin beta-2A chain",
  "gene": "UniProtKB:Q13885",
  "term_id": "GO:0005737",
  "gene_symbol": "TUBB2A"
}